{
  "term_label": "cell-cell junction organization",
  "gene_name": "LIM and senescent cell antigen-like-containing domain protein 2",
  "term_id": "GO:0045216",
  "gene_symbol": "LIMS2",
  "gene": "UniProtKB:Q7Z4I7"
}